{
  "gene_name": "Signal transducer and activator of transcription 3",
  "term_label": "growth hormone receptor signaling pathway via JAK-STAT",
  "gene_symbol": "STAT3",
  "gene": "UniProtKB:P40763",
  "term_id": "GO:0060397"
}